{
  "term_label": "protein phosphatase 1 binding",
  "term_id": "GO:0008157",
  "gene_symbol": "PPP1R3G",
  "gene": "UniProtKB:B7ZBB8",
  "gene_name": "Protein phosphatase 1 regulatory subunit 3G"
}